{
  "term_label": "protein serine/threonine kinase activity",
  "term_id": "GO:0004674",
  "gene_name": "Microtubule-associated serine_threonine-protein kinase 4",
  "gene_symbol": "MAST4",
  "gene": "UniProtKB:O15021"
}